{
  "term_label": "nucleus",
  "gene_symbol": "THAP2",
  "term_id": "GO:0005634",
  "gene_name": "THAP domain-containing protein 2",
  "gene": "UniProtKB:Q9H0W7"
}